positive regulation of phialide development [GO:0070807] (biological process) Sources: GOC:mah Definition: Any process that activates or increases the frequency, rate or extent of phialide development, a process that leads to the formation of phialides. Phialides are specialized cells that bud from the ends of metulae on the conidiophore tip. Relationships: is a type of positive regulation of cell development [GO:0010720]; is a type of GO:0070805; is a type of positive regulation of reproductive process [GO:2000243]; positively regulates phialide development [GO:0070790]